{
  "term_label": "receptor antagonist activity",
  "gene_name": "Humanin-like 2",
  "gene": "UniProtKB:P0CJ69",
  "gene_symbol": "MTRNR2L2",
  "term_id": "GO:0048019"
}